{
  "gene": "UniProtKB:Q9NRX6",
  "gene_name": "Protein kish-B",
  "term_label": "Unknown cellular component",
  "gene_symbol": "TMEM167B",
  "term_id": "UNKNOWN:0003"
}